{
  "gene_symbol": "SYT6",
  "term_id": "GO:0005886",
  "gene": "UniProtKB:Q5T7P8",
  "term_label": "plasma membrane",
  "gene_name": "Synaptotagmin-6"
}